{
  "gene_symbol": "MYOCOS",
  "gene_name": "Myocilin opposite strand protein",
  "term_label": "Unknown molecular function",
  "term_id": "UNKNOWN:0001",
  "gene": "UniProtKB:A0A1B0GUC4"
}